purine deoxyribonucleoside biosynthetic process [GO:0046123] (biological process) Sources: GOC:ai Definition: The chemical reactions and pathways resulting in the formation of any purine deoxyribonucleoside, one of a family of organic molecules consisting of a purine base covalently bonded to a sugar deoxyribose (a deoxyribonucleoside). Relationships: is a type of purine nucleoside biosynthetic process [GO:0042451]; is a type of deoxyribonucleoside biosynthetic process [GO:0046120]; is a type of GO:0046122 Subtypes: deoxyguanosine biosynthetic process [GO:0042452], purine deoxyribonucleoside salvage [GO:0043098], GO:0046091, deoxyinosine biosynthetic process [GO:0046095] Also known as: purine deoxyribonucleoside anabolism, purine deoxyribonucleoside biosynthesis, purine deoxyribonucleoside formation, purine deoxyribonucleoside synthesis